{
  "gene": "UniProtKB:Q8WUJ0",
  "term_id": "GO:0062026",
  "term_label": "negative regulation of SCF-dependent proteasomal ubiquitin-dependent catabolic process",
  "gene_name": "Serine_threonine_tyrosine-interacting protein",
  "gene_symbol": "STYX"
}